{
  "term_label": "Unknown molecular function",
  "gene_symbol": "NAT16",
  "gene_name": "Probable N-acetyltransferase 16",
  "term_id": "UNKNOWN:0001",
  "gene": "UniProtKB:Q8N8M0"
}